{
  "gene_symbol": "RC3H2",
  "term_label": "protein polyubiquitination",
  "gene_name": "Roquin-2",
  "term_id": "GO:0000209",
  "gene": "UniProtKB:Q9HBD1"
}